colon epithelial cell chemotaxis [GO:0061583] (biological process) Definition: The directed movement of a colon epithelial cell guided by a specific chemical concentration gradient. Movement may be towards a higher concentration (positive chemotaxis) or towards a lower concentration (negative chemotaxis). Sources: GOC:dph Relationships: is_a cell chemotaxis [GO:0060326]; is a type of GO:0061580